{
  "term_id": "GO:0005814",
  "gene_name": "Centrin-2",
  "gene": "UniProtKB:P41208",
  "gene_symbol": "CETN2",
  "term_label": "centriole"
}